{
  "gene_name": "Hairy and enhancer of split-related protein HELT",
  "gene": "UniProtKB:A6NFD8",
  "term_label": "anterior/posterior pattern specification",
  "gene_symbol": "HELT",
  "term_id": "GO:0009952"
}